methyl-CpG binding [GO:0008327] (molecular function) Definition: Binding to a methylated cytosine/guanine dinucleotide. References: PMID:11746232 Sources: GOC:jl Relationships: is a type of nucleotide binding [GO:0000166]; is a type of GO:0043565